{
  "term_label": "spermatogenesis",
  "gene_name": "Ribosomal protein uL16-like",
  "term_id": "GO:0007283",
  "gene_symbol": "RPL10L",
  "gene": "UniProtKB:Q96L21"
}